meiotic cell cycle checkpoint signaling [GO:0033313] (biological process) Relationships: is a type of cell cycle checkpoint signaling [GO:0000075]; is a type of GO:1903046 Also known as: meiotic cell cycle checkpoint, signal transduction involved in meiotic cell cycle checkpoint Subtypes: meiotic DNA integrity checkpoint signaling [GO:0044778], meiotic spindle checkpoint signaling [GO:0044779], meiotic recombination checkpoint signaling [GO:0051598] Definition: A signaling process that contributes to a meiotic cell cycle checkpoint that ensures accurate chromosome replication and segregation by preventing progression through a meiotic cell cycle until conditions are suitable for the cell to proceed to the next stage. Sources: GOC:mtg_cell_cycle